{
  "term_label": "cytoplasm",
  "gene_name": "Sulfotransferase 1A2",
  "term_id": "GO:0005737",
  "gene_symbol": "SULT1A2",
  "gene": "UniProtKB:P50226"
}